purine nucleotide biosynthetic process [GO:0006164] (biological process) Definition: The chemical reactions and pathways resulting in the formation of a purine nucleotide, a compound consisting of nucleoside (a purine base linked to a deoxyribose or ribose sugar) esterified with a phosphate group at either the 3' or 5'-hydroxyl group of the sugar. Regulation: regulated by GO:1900371; negatively regulated by negative regulation of purine nucleotide biosynthetic process [GO:1900372]; positively regulated by positive regulation of purine nucleotide biosynthetic process [GO:1900373] Subtypes: NADP+ biosynthetic process [GO:0006741], purine ribonucleotide biosynthetic process [GO:0009152], purine deoxyribonucleotide biosynthetic process [GO:0009153], NAD+ biosynthetic process [GO:0009435], purine nucleotide salvage [GO:0032261] Relationships: is a type of GO:0006163; is a type of GO:0009165; is a type of GO:0072522 Also known as: purine nucleotide anabolism, purine nucleotide biosynthesis, purine nucleotide formation, purine nucleotide synthesis Sources: GOC:go_curators, ISBN:0198506732